{
  "gene_symbol": "POLL",
  "gene": "UniProtKB:Q9UGP5",
  "gene_name": "DNA polymerase lambda",
  "term_label": "DNA-directed DNA polymerase activity",
  "term_id": "GO:0003887"
}